regulation of organic acid transport [GO:0032890] (biological process) Definition: Any process that modulates the frequency, rate or extent of the directed movement of organic acids into, out of or within a cell, or between cells, by means of some agent such as a transporter or pore. Sources: GOC:mah Relationships: is_a GO:0051049; regulates organic acid transport [GO:0015849] Subtypes: regulation of L-glutamate import across plasma membrane [GO:0002036], regulation of glutamate secretion [GO:0014048], regulation of gamma-aminobutyric acid secretion [GO:0014052], negative regulation of organic acid transport [GO:0032891], positive regulation of organic acid transport [GO:0032892], regulation of gluconate transmembrane transport [GO:0035430], regulation of gamma-aminobutyric acid uptake involved in transmission of nerve impulse [GO:0051947], regulation of proline transport [GO:0070881], regulation of bile acid secretion [GO:0120188], regulation of D-aspartate import across plasma membrane [GO:0140215], GO:1900923, regulation of L-threonine import across plasma membrane [GO:1900926], regulation of L-tyrosine import across plasma membrane [GO:1900929], regulation of proline import across plasma membrane [GO:1902834], GO:1904448, GO:1904624, regulation of L-lysine import across plasma membrane [GO:1905008], GO:1905532, regulation of L-arginine import across plasma membrane [GO:1905541], regulation of L-methionine import across plasma membrane [GO:1905624], regulation of fatty acid transport [GO:2000191], regulation of glutamine transport [GO:2000485]